{
  "gene_name": "Piwi-like protein 2",
  "term_label": "piRNA binding",
  "gene": "UniProtKB:Q8TC59",
  "term_id": "GO:0034584",
  "gene_symbol": "PIWIL2"
}